{
  "gene": "UniProtKB:Q9NYK6",
  "gene_name": "Protein EURL homolog",
  "term_label": "Unknown molecular function",
  "term_id": "UNKNOWN:0001",
  "gene_symbol": "EURL"
}